{
  "term_label": "cytoplasm",
  "term_id": "GO:0005737",
  "gene_symbol": "PPIA",
  "gene_name": "Peptidyl-prolyl cis-trans isomerase A",
  "gene": "UniProtKB:P62937"
}